{
  "gene_name": "Protein kinase C and casein kinase substrate in neurons protein 2",
  "term_label": "endosome",
  "gene_symbol": "PACSIN2",
  "term_id": "GO:0005768",
  "gene": "UniProtKB:Q9UNF0"
}